{
  "gene_symbol": "CMKLR1",
  "term_id": "GO:0006954",
  "term_label": "inflammatory response",
  "gene": "UniProtKB:Q99788",
  "gene_name": "Chemerin-like receptor 1"
}